{
  "term_label": "plasma membrane",
  "gene_name": "CD166 antigen",
  "gene": "UniProtKB:Q13740",
  "gene_symbol": "ALCAM",
  "term_id": "GO:0005886"
}